{
  "term_label": "negative regulation of angiogenesis",
  "gene": "UniProtKB:O00522",
  "gene_symbol": "KRIT1",
  "gene_name": "Krev interaction trapped protein 1",
  "term_id": "GO:0016525"
}